{
  "gene": "UniProtKB:Q9BXY5",
  "term_label": "Unknown biological process",
  "gene_name": "Calcyphosin-2",
  "term_id": "UNKNOWN:0002",
  "gene_symbol": "CAPS2"
}